N-acetylglucosamine metabolic process [GO:0006044] (biological process) Relationships: is a type of amino sugar metabolic process [GO:0006040] Sources: ISBN:0198506732 Subtypes: N-acetylglucosamine biosynthetic process [GO:0006045], N-acetylglucosamine catabolic process [GO:0006046] Definition: The chemical reactions and pathways involving N-acetylglucosamine. The D isomer is a common structural unit of glycoproteins in plants, bacteria and animals; it is often the terminal sugar of an oligosaccharide group of a glycoprotein. Also known as: N-acetylglucosamine metabolism